{
  "gene_name": "Autophagy protein 5",
  "gene": "UniProtKB:Q9H1Y0",
  "term_id": "GO:0034727",
  "gene_symbol": "ATG5",
  "term_label": "piecemeal microautophagy of the nucleus"
}